{
  "term_label": "endoplasmic reticulum membrane",
  "term_id": "GO:0005789",
  "gene_name": "2-acylglycerol O-acyltransferase 3",
  "gene": "UniProtKB:Q86VF5",
  "gene_symbol": "MOGAT3"
}